{
  "gene_symbol": "HSBP1L1",
  "gene": "UniProtKB:C9JCN9",
  "term_label": "cellular heat acclimation",
  "gene_name": "Heat shock factor-binding protein 1-like protein 1",
  "term_id": "GO:0070370"
}